{
  "term_id": "UNKNOWN:0002",
  "gene_name": "Putative aldo-keto reductase family 1 member C8",
  "term_label": "Unknown biological process",
  "gene_symbol": "AKR1C8",
  "gene": "UniProtKB:Q5T2L2"
}